positive regulation of convergent extension involved in gastrulation [GO:1904105] (biological process) References: PMID:24892953 Sources: GOC:TermGenie, GOC:dph, GO_REF:0000058 Subtypes: positive regulation of convergent extension involved in somitogenesis [GO:1904129], GO:1904132, GO:1904135, GO:1904138 Relationships: is a type of GO:1904103; is a type of positive regulation of morphogenesis of an epithelium [GO:1905332]; positively regulates convergent extension involved in gastrulation [GO:0060027] Also known as: up regulation of convergent extension involved in gastrulation, up-regulation of convergent extension involved in gastrulation, upregulation of convergent extension involved in gastrulation, activation of convergent extension involved in gastrulation Definition: Any process that activates or increases the frequency, rate or extent of convergent extension involved in gastrulation.